{
  "term_label": "Unknown cellular component",
  "gene_symbol": "CCDC27",
  "gene_name": "Coiled-coil domain-containing protein 27",
  "gene": "UniProtKB:Q2M243",
  "term_id": "UNKNOWN:0003"
}